{
  "term_label": "plasma membrane",
  "term_id": "GO:0005886",
  "gene_symbol": "OR56B1",
  "gene_name": "Olfactory receptor 56B1",
  "gene": "UniProtKB:Q8NGI3"
}